chemokine (C-C motif) ligand 5 production [GO:0071609] (BP) Also known as: CCL5 production, RANTES production, Regulated upon Activation, Normal T-cell Expressed, and Secreted production Relationships: is a type of chemokine production [GO:0032602] Regulation: regulated by GO:0071649; negatively regulated by GO:0071650; positively regulated by positive regulation of chemokine (C-C motif) ligand 5 production [GO:0071651] Definition: The appearance of chemokine (C-C motif) ligand 5 due to biosynthesis or secretion following a cellular stimulus, resulting in an increase in its intracellular or extracellular levels. Sources: GOC:add, GOC:rv